memory [GO:0007613] (biological process) Sources: GOC:curators, ISBN:0582227089 Subtypes: short-term memory [GO:0007614], anesthesia-resistant memory [GO:0007615], long-term memory [GO:0007616], medium-term memory [GO:0072375] Definition: The activities involved in the mental information processing system that receives (registers), modifies, stores, and retrieves informational stimuli. The main stages involved in the formation and retrieval of memory are encoding (processing of received information by acquisition), storage (building a permanent record of received information as a result of consolidation) and retrieval (calling back the stored information and use it in a suitable way to execute a given task). Relationships: is a type of GO:0007611